{
  "gene": "UniProtKB:Q9H813",
  "gene_symbol": "PACC1",
  "term_id": "UNKNOWN:0003",
  "gene_name": "Proton-activated chloride channel",
  "term_label": "Unknown cellular component"
}